mitotic cell size control checkpoint signaling [GO:0031567] (BP) Sources: GOC:mtg_cell_cycle Definition: A signal transduction process that contributes to a cell size control checkpoint during mitosis. Also known as: mitotic cell cycle cell size control checkpoint, mitotic cell size control checkpoint, signal transduction involved in cell size control checkpoint Relationships: is a type of mitotic cell cycle checkpoint signaling [GO:0007093]; is a type of negative regulation of mitotic cell cycle phase transition [GO:1901991] Subtypes: mitotic G1 cell size control checkpoint signaling [GO:0031568], mitotic G2 cell size control checkpoint signaling [GO:0031569]